{
  "term_id": "UNKNOWN:0002",
  "gene_name": "Putative uncharacterized protein PRO1716",
  "gene": "UniProtKB:Q9UHU1",
  "gene_symbol": "PRO1716",
  "term_label": "Unknown biological process"
}